phagophore assembly site [GO:0000407] (cellular component) References: PMID:11689437, PMID:12048214, PMID:12554655 Sources: GOC:elh Also known as: PAS, perivacuolar space, pre-autophagosomal structure Relationships: is a type of cellular anatomical structure [GO:0110165]; is part of GO:0005737 Definition: Punctate structures proximal to the endoplasmic reticulum which are the sites where the Atg machinery assembles upon autophagy induction.